{
  "gene_name": "TATA-box-binding protein-associated factor 11-like protein 12",
  "term_id": "GO:0051123",
  "gene_symbol": "TAF11L12",
  "gene": "UniProtKB:A0A1W2PPW3",
  "term_label": "RNA polymerase II preinitiation complex assembly"
}